positive regulation of antifungal innate immune response [GO:1905036] (biological process) Also known as: up regulation of antifungal innate immune response, up-regulation of antifungal innate immune response, upregulation of antifungal innate immune response, activation of antifungal innate immune response Definition: Any process that activates or increases the frequency, rate or extent of an antifungal innate immune response. Relationships: is a type of positive regulation of innate immune response [GO:0045089]; is a type of regulation of antifungal innate immune response [GO:1905034]; positively regulates antifungal innate immune response [GO:0061760] References: PMID:22470487 Sources: GOC:TermGenie, GOC:dph, GO_REF:0000058